{
  "gene_name": "Killer cell immunoglobulin-like receptor 2DS3",
  "gene": "UniProtKB:Q14952",
  "term_id": "GO:0005886",
  "term_label": "plasma membrane",
  "gene_symbol": "KIR2DS3"
}